hydroxymethylbilane synthase activity [GO:0004418] (molecular function) Also known as: uroporphyrinogen I synthase activity, uroporphyrinogen I synthetase activity, (4-(2-carboxyethyl)-3-(carboxymethyl)pyrrol-2-yl)methyltransferase (hydrolyzing) activity, (4-[2-carboxyethyl]-3-[carboxymethyl]pyrrol-2-yl)methyltransferase (hydrolysing), HMB-synthase activity, porphobilinogen ammonia-lyase (polymerizing), porphobilinogen deaminase activity, porphobilinogen:(4-[2-carboxyethyl]-3-[carboxymethyl]pyrrol-2-yl)methyltransferase (hydrolysing), pre-uroporphyrinogen synthase activity, uroporphyrinogen synthase activity, uroporphyrinogen synthetase activity Sources: EC:2.5.1.61, RHEA:13185 Definition: Catalysis of the reaction: H2O + 4 porphobilinogen = hydroxymethylbilane + 4 NH4. Relationships: is a type of GO:0016765